{
  "gene_symbol": "PMS2CL",
  "gene": "UniProtKB:Q68D20",
  "gene_name": "Protein PMS2CL",
  "term_label": "Unknown molecular function",
  "term_id": "UNKNOWN:0001"
}